{
  "gene": "UniProtKB:O95721",
  "term_label": "SNAP receptor activity",
  "gene_symbol": "SNAP29",
  "gene_name": "Synaptosomal-associated protein 29",
  "term_id": "GO:0005484"
}